negative regulation of response to salt stress [GO:1901001] (biological process) References: PMID:22627139 Sources: GOC:TermGenie Relationships: is a type of negative regulation of response to stimulus [GO:0048585]; is_a regulation of response to salt stress [GO:1901000]; negatively regulates response to salt stress [GO:0009651] Also known as: down regulation of response to ionic osmotic stress, down regulation of response to salt stress, down regulation of salinity response, down-regulation of response to ionic osmotic stress, down-regulation of response to salt stress, down-regulation of salinity response, downregulation of response to ionic osmotic stress, downregulation of response to salt stress, downregulation of salinity response, inhibition of response to ionic osmotic stress, inhibition of salinity response, negative regulation of response to ionic osmotic stress, negative regulation of salinity response, inhibition of response to salt stress Definition: Any process that stops, prevents or reduces the frequency, rate or extent of response to salt stress. Subtypes: negative regulation of cellular hyperosmotic salinity response [GO:1900070]